{
  "gene_name": "DnaJ homolog subfamily C member 14",
  "gene_symbol": "DNAJC14",
  "term_id": "UNKNOWN:0003",
  "gene": "UniProtKB:Q6Y2X3",
  "term_label": "Unknown cellular component"
}